{
  "term_id": "GO:0008508",
  "gene_symbol": "SLC10A1",
  "gene_name": "Hepatic sodium_bile acid cotransporter",
  "gene": "UniProtKB:Q14973",
  "term_label": "bile acid:sodium symporter activity"
}